positive regulation of uracil import across plasma membrane [GO:1905531] (BP) Definition: Any process that activates or increases the frequency, rate or extent of uracil import across plasma membrane. Relationships: is_a positive regulation of transmembrane transport [GO:0034764]; is a type of regulation of uracil import across plasma membrane [GO:1905529]; positively regulates uracil import across plasma membrane [GO:0098721] References: PMID:26536126 Sources: GOC:TermGenie, GO_REF:0000058